heme transmembrane transporter activity [GO:0015232] (molecular function) References: PMID:29549126 Definition: Enables the transfer of heme from one side of a membrane to the other. Relationships: is a type of transmembrane transporter activity [GO:0022857]; is part of heme transport [GO:0015886] Also known as: heme transporter activity, haem transporter activity Subtypes: GO:0015439, heme B transmembrane transporter activity [GO:0170003]